JUN kinase kinase activity [GO:0008545] (molecular function) References: PMID:11057897, PMID:11790549 Sources: GOC:bf Definition: Catalysis of the phosphorylation of tyrosine and threonine residues in a c-Jun NH2-terminal kinase (JNK), a member of a subgroup of mitogen-activated protein kinases (MAPKs), which signal in response to cytokines and exposure to environmental stress. JUN kinase kinase (JNKK) is a dual-specificity protein kinase kinase and requires activation by a serine/threonine kinase JUN kinase kinase kinase. Relationships: is a type of GO:0004708; is part of JNK cascade [GO:0007254] Also known as: JNKK